phospholipase D activity [GO:0004630] (molecular function) Relationships: is a type of phospholipase activity [GO:0004620]; is a type of phosphoric diester hydrolase activity [GO:0008081] Also known as: choline phosphatase activity, lecithinase D activity, lipophosphodiesterase II activity, phosphatidylcholine phosphatidohydrolase activity Regulation: negatively regulated by phospholipase D inhibitor activity [GO:0060961]; positively regulated by phospholipase D activator activity [GO:1990583] Subtypes: glycosylphosphatidylinositol phospholipase D activity [GO:0004621] Definition: Catalysis of the reaction: a phosphatidylcholine + H2O = choline + a phosphatidate. Sources: EC:3.1.4.4